{
  "gene": "UniProtKB:A8MTL3",
  "term_id": "GO:0000795",
  "term_label": "synaptonemal complex",
  "gene_name": "RING finger protein 212B",
  "gene_symbol": "RNF212B"
}